{
  "gene_name": "Cleavage and polyadenylation specificity factor subunit 2",
  "gene": "UniProtKB:Q9P2I0",
  "term_label": "mRNA cleavage and polyadenylation specificity factor complex",
  "gene_symbol": "CPSF2",
  "term_id": "GO:0005847"
}